symbiont-mediated disruption of host phagosome [GO:0141160] (BP) Relationships: is_a symbiont-mediated disruption of host cellular anatomical structure [GO:0052008] Definition: The process in which an organism effects a change that impairs the structure or function of host phagosomes. References: PMID:15487949, PMID:21412437, PMID:30057173